{
  "gene": "UniProtKB:Q9NS87",
  "gene_symbol": "KIF15",
  "term_id": "GO:0007018",
  "term_label": "microtubule-based movement",
  "gene_name": "Kinesin-like protein KIF15"
}